{
  "term_id": "GO:0005634",
  "gene_name": "Ras-related GTP-binding protein C",
  "term_label": "nucleus",
  "gene": "UniProtKB:Q9HB90",
  "gene_symbol": "RRAGC"
}